2-keto-3-deoxy-L-rhamnonate aldolase activity [GO:0106099] (molecular function) References: PMID:18754683 Sources: EC:4.1.2.53, GOC:imk Definition: Catalysis of the reaction 2-dehydro-3-deoxy-L-rhamnonate = pyruvate + (S)-lactaldehyde. Relationships: is a type of GO:0016832